{
  "term_label": "mRNA splice site recognition",
  "gene_symbol": "CELF3",
  "gene": "UniProtKB:Q5SZQ8",
  "gene_name": "CUGBP Elav-like family member 3",
  "term_id": "GO:0006376"
}